N-(5-amino-5-carboxypentanoyl)-L-cysteinyl-D-valine synthase activity [GO:0050564] (molecular function) Definition: Catalysis of the reaction: L-2-aminoadipate + L-cysteine + L-valine + 3 ATP + H2O = N-[(5S)-5-amino-5-carboxypentanoyl]-L-cysteinyl-D-valine + 3 AMP + 3 diphosphate + 6 H+. Relationships: is a type of acid-amino acid ligase activity [GO:0016881] Sources: EC:6.3.2.26, RHEA:23196 Also known as: ACV synthetase activity, delta-(L-alpha-aminoadipyl)-L-cysteinyl-D-valine synthetase activity, L-2-aminohexanedioate:L-cysteine:L-valine ligase (AMP-forming, valine-inverting), L-alpha-aminoadipyl-cysteinyl-valine synthetase activity, L-delta-(alpha-aminoadipoyl)-L-cysteinyl-D-valine synthetase activity